{
  "gene_name": "Adhesion G protein-coupled receptor A3",
  "term_label": "external side of plasma membrane",
  "term_id": "GO:0009897",
  "gene_symbol": "ADGRA3",
  "gene": "UniProtKB:Q8IWK6"
}